{
  "gene_symbol": "SSU72L3",
  "term_id": "GO:0005847",
  "gene": "UniProtKB:A0A1W2PQJ5",
  "term_label": "mRNA cleavage and polyadenylation specificity factor complex",
  "gene_name": "RNA polymerase II subunit A C-terminal domain phosphatase SSU72 like protein 3"
}